{
  "term_id": "GO:0042981",
  "gene": "UniProtKB:O43423",
  "gene_name": "Putative uncharacterized protein ANP32CP",
  "gene_symbol": "ANP32CP",
  "term_label": "regulation of apoptotic process"
}